atrioventricular node cell fate commitment [GO:0060929] (biological process) Sources: GOC:mtg_heart Also known as: AV node cell fate commitment Definition: The commitment of cells to atrioventricular (AV) node cell fates and their capacity to differentiate into AV node cells. Relationships: is a type of cardiac pacemaker cell fate commitment [GO:0060927]; is part of atrioventricular node cell differentiation [GO:0060922]